{
  "term_label": "Unknown cellular component",
  "gene_name": "Protein RD3-like",
  "term_id": "UNKNOWN:0003",
  "gene_symbol": "RD3L",
  "gene": "UniProtKB:P0DJH9"
}